{
  "term_id": "UNKNOWN:0002",
  "gene_name": "Translin-associated protein X",
  "gene_symbol": "TSNAX",
  "gene": "UniProtKB:Q99598",
  "term_label": "Unknown biological process"
}